{
  "gene_name": "Putative uncharacterized protein ARHGAP5-AS1",
  "term_label": "Unknown biological process",
  "gene": "UniProtKB:Q96IT6",
  "gene_symbol": "ARHGAP5-AS1",
  "term_id": "UNKNOWN:0002"
}